{
  "gene_name": "Transmembrane protein 196",
  "term_label": "Unknown cellular component",
  "term_id": "UNKNOWN:0003",
  "gene": "UniProtKB:Q5HYL7",
  "gene_symbol": "TMEM196"
}